{
  "term_label": "neuropeptide binding",
  "gene_symbol": "PTGDR2",
  "term_id": "GO:0042923",
  "gene": "UniProtKB:Q9Y5Y4",
  "gene_name": "Prostaglandin D2 receptor 2"
}